maintenance of Golgi location [GO:0051684] (biological process) Definition: Any process in which the Golgi is maintained in a specific location within a cell and prevented from moving elsewhere. Relationships: is a type of Golgi localization [GO:0051645]; is a type of maintenance of organelle location [GO:0051657] Also known as: maintenance of Golgi apparatus localization, maintenance of Golgi body localization, maintenance of Golgi localization Sources: GOC:ai, GOC:dph, GOC:tb